{
  "term_id": "UNKNOWN:0001",
  "gene": "UniProtKB:Q5JPF3",
  "term_label": "Unknown molecular function",
  "gene_name": "Ankyrin repeat domain-containing protein 36C",
  "gene_symbol": "ANKRD36C"
}